{
  "gene_name": "LysM and putative peptidoglycan-binding domain-containing protein 4",
  "gene": "UniProtKB:Q5XG99",
  "term_id": "UNKNOWN:0001",
  "gene_symbol": "LYSMD4",
  "term_label": "Unknown molecular function"
}